{
  "gene_symbol": "REG3G",
  "term_label": "hormone activity",
  "gene": "UniProtKB:Q6UW15",
  "term_id": "GO:0005179",
  "gene_name": "Regenerating islet-derived protein 3-gamma"
}